{
  "term_id": "GO:0007169",
  "gene_symbol": "SRMS",
  "term_label": "cell surface receptor protein tyrosine kinase signaling pathway",
  "gene": "UniProtKB:Q9H3Y6",
  "gene_name": "Tyrosine-protein kinase Srms"
}